{
  "term_id": "GO:0016192",
  "gene_name": "ADP-ribosylation factor-like protein 4A",
  "gene": "UniProtKB:P40617",
  "gene_symbol": "ARL4A",
  "term_label": "vesicle-mediated transport"
}